icosahedral viral capsid, neck fiber [GO:0098033] (cellular component) Sources: GOC:bm Definition: A fiber attached to the neck at the base of some icosahedral viral capsids. Relationships: is a type of viral capsid, fiber [GO:0098022]; is part of GO:0098030